{
  "gene_symbol": "THAP2",
  "term_id": "UNKNOWN:0002",
  "gene_name": "THAP domain-containing protein 2",
  "term_label": "Unknown biological process",
  "gene": "UniProtKB:Q9H0W7"
}